{
  "gene": "UniProtKB:P01286",
  "term_label": "growth hormone secretion",
  "gene_symbol": "GHRH",
  "term_id": "GO:0030252",
  "gene_name": "Somatoliberin"
}